{
  "gene": "UniProtKB:Q09028",
  "gene_name": "Histone-binding protein RBBP4",
  "gene_symbol": "RBBP4",
  "term_label": "regulation of DNA-templated transcription",
  "term_id": "GO:0006355"
}